{
  "term_label": "Unknown cellular component",
  "gene_name": "Ribosomal protein eL22-like",
  "term_id": "UNKNOWN:0003",
  "gene_symbol": "RPL22L1",
  "gene": "UniProtKB:Q6P5R6"
}